{
  "term_label": "RNA polymerase II complex binding",
  "term_id": "GO:0000993",
  "gene_name": "Regulation of nuclear pre-mRNA domain-containing protein 2",
  "gene": "UniProtKB:Q5VT52",
  "gene_symbol": "RPRD2"
}